{
  "term_label": "centrosome",
  "gene": "UniProtKB:Q9NVX0",
  "gene_symbol": "HAUS2",
  "term_id": "GO:0005813",
  "gene_name": "HAUS augmin-like complex subunit 2"
}